{
  "term_id": "GO:0005737",
  "gene": "UniProtKB:P09543",
  "term_label": "cytoplasm",
  "gene_name": "2',3'-cyclic-nucleotide 3'-phosphodiesterase",
  "gene_symbol": "CNP"
}